{
  "gene": "UniProtKB:Q6PI98",
  "term_label": "chromatin remodeling",
  "gene_name": "INO80 complex subunit C",
  "term_id": "GO:0006338",
  "gene_symbol": "INO80C"
}